{
  "gene_symbol": "Q8N3U1",
  "gene": "UniProtKB:Q8N3U1",
  "gene_name": "Putative uncharacterized protein LOC400692",
  "term_id": "UNKNOWN:0002",
  "term_label": "Unknown biological process"
}